{
  "term_id": "GO:0045089",
  "term_label": "positive regulation of innate immune response",
  "gene_name": "Phospholipid scramblase 2",
  "gene_symbol": "PLSCR2",
  "gene": "UniProtKB:Q9NRY7"
}